{
  "gene_name": "Serine_threonine-protein kinase VRK1",
  "gene": "UniProtKB:Q99986",
  "term_id": "GO:0006974",
  "term_label": "DNA damage response",
  "gene_symbol": "VRK1"
}